{
  "term_id": "GO:0030295",
  "gene_symbol": "MOB3A",
  "term_label": "protein kinase activator activity",
  "gene_name": "MOB kinase activator 3A",
  "gene": "UniProtKB:Q96BX8"
}